{
  "gene": "UniProtKB:Q9NRZ7",
  "gene_name": "1-acyl-sn-glycerol-3-phosphate acyltransferase gamma",
  "term_label": "Unknown biological process",
  "gene_symbol": "AGPAT3",
  "term_id": "UNKNOWN:0002"
}